ketol-acid reductoisomerase activity [GO:0004455] (molecular function) Definition: Catalysis of the reaction: (R)-2,3-dihydroxy-3-methylbutanoate + NADP+ = (S)-2-hydroxy-2-methyl-3-oxobutanoate + NADPH + H+. Sources: EC:1.1.1.86 Also known as: (R)-2,3-dihydroxy-3-methylbutanoate:NADP+ oxidoreductase (isomerizing), 2-hydroxy-3-keto acid reductoisomerase activity, acetohydroxy acid isomeroreductase activity, acetohydroxy acid reductoisomerase activity, acetolactate reductoisomerase activity, alpha-keto-beta-hydroxylacyl reductoisomerase activity, dihydroxyisovalerate (isomerizing) dehydrogenase activity, dihydroxyisovalerate dehydrogenase (isomerizing) activity, isomeroreductase activity, ketol acid reductoisomerase activity, reductoisomerase activity Relationships: is a type of oxidoreductase activity, acting on the CH-OH group of donors, NAD or NADP as acceptor [GO:0016616]